{
  "gene": "UniProtKB:P20393",
  "gene_name": "Nuclear receptor subfamily 1 group D member 1",
  "term_id": "GO:0000122",
  "term_label": "negative regulation of transcription by RNA polymerase II",
  "gene_symbol": "NR1D1"
}